positive regulation of mast cell apoptotic process [GO:0033027] (BP) Also known as: up regulation of mast cell apoptosis, up-regulation of mast cell apoptosis, upregulation of mast cell apoptosis, activation of mast cell apoptosis, positive regulation of mast cell apoptosis, stimulation of mast cell apoptosis Relationships: is a type of positive regulation of immune system process [GO:0002684]; is a type of GO:0033025; is_a positive regulation of myeloid cell apoptotic process [GO:0033034]; is a type of positive regulation of leukocyte apoptotic process [GO:2000108]; positively regulates GO:0033024 Definition: Any process that activates or increases the frequency, rate, or extent of mast cell apoptotic process. Sources: GOC:add, GOC:mtg_apoptosis